dethiobiotin import across plasma membrane [GO:1905136] (biological process) Also known as: dethiobiotin import into cell, dethiobiotin import Definition: The directed movement of dethiobiotin from outside of a cell, across the plasma membrane and into the cytosol. Relationships: is a type of monocarboxylic acid transport [GO:0015718]; is a type of GO:0042886; is a type of import across plasma membrane [GO:0098739]; is a type of carboxylic acid transmembrane transport [GO:1905039] References: PMID:12557275 Sources: GOC:TermGenie, GO_REF:0000075